{
  "term_id": "UNKNOWN:0002",
  "gene": "UniProtKB:Q5J8M3",
  "gene_symbol": "EMC4",
  "term_label": "Unknown biological process",
  "gene_name": "ER membrane protein complex subunit 4"
}